{
  "gene_symbol": "PLP1",
  "term_label": "axon development",
  "gene": "UniProtKB:P60201",
  "gene_name": "Myelin proteolipid protein",
  "term_id": "GO:0061564"
}